{
  "term_label": "execution phase of apoptosis",
  "gene_name": "Bcl-2-binding component 3, isoforms 3_4",
  "term_id": "GO:0097194",
  "gene": "UniProtKB:Q96PG8",
  "gene_symbol": "BBC3"
}